{
  "term_label": "presynaptic membrane",
  "term_id": "GO:0042734",
  "gene_name": "Adhesion G protein-coupled receptor L1",
  "gene_symbol": "ADGRL1",
  "gene": "UniProtKB:O94910"
}